{
  "term_id": "GO:0060291",
  "gene": "UniProtKB:O43566",
  "term_label": "long-term synaptic potentiation",
  "gene_name": "Regulator of G-protein signaling 14",
  "gene_symbol": "RGS14"
}